{
  "gene": "UniProtKB:Q9NZD8",
  "term_id": "GO:0005829",
  "gene_name": "Maspardin",
  "gene_symbol": "SPG21",
  "term_label": "cytosol"
}